protein kinase activity [GO:0004672] (molecular function) Relationships: is a type of GO:0016301; is a type of phosphotransferase activity, alcohol group as acceptor [GO:0016773]; is a type of catalytic activity, acting on a protein [GO:0140096] Regulation: negatively regulated by protein kinase inhibitor activity [GO:0004860]; negatively regulated by negative regulation of protein kinase activity [GO:0006469]; regulated by GO:0019887; positively regulated by protein kinase activator activity [GO:0030295]; regulated by regulation of protein kinase activity [GO:0045859]; positively regulated by positive regulation of protein kinase activity [GO:0045860] Definition: Catalysis of the phosphorylation of an amino acid residue in a protein, usually according to the reaction: a protein + ATP = a phosphoprotein + ADP. Also known as: protamine kinase activity References: PMID:25399640 Note: Note that triphosphate is used as a phosphate donor by at least one kinase. Subtypes: protein histidine kinase activity [GO:0004673], protein serine/threonine kinase activity [GO:0004674], protein serine/threonine/tyrosine kinase activity [GO:0004712], protein tyrosine kinase activity [GO:0004713], histidine phosphotransfer kinase activity [GO:0009927], transmembrane receptor protein kinase activity [GO:0019199], histone kinase activity [GO:0035173], beta-adrenergic receptor kinase activity [GO:0047696], cyclin-dependent protein kinase activity [GO:0097472], GO:0106264, protein serine kinase activity [GO:0106310], protein arginine kinase activity [GO:1990424]